{
  "gene": "UniProtKB:P10912",
  "gene_symbol": "GHR",
  "term_label": "external side of plasma membrane",
  "gene_name": "Growth hormone receptor",
  "term_id": "GO:0009897"
}